oleate transmembrane transporter activity [GO:1901480] (molecular function) Definition: Enables the transfer of oleate from one side of a membrane to the other. Relationships: is_a GO:0005324 Also known as: oleate transporter activity References: PMID:19493158 Sources: GOC:TermGenie